{
  "term_id": "UNKNOWN:0001",
  "gene": "UniProtKB:Q9H8W2",
  "term_label": "Unknown molecular function",
  "gene_symbol": "LINC00472",
  "gene_name": "Putative uncharacterized protein encoded by LINC00472"
}